{
  "gene": "UniProtKB:Q9GZQ8",
  "term_id": "GO:0000421",
  "term_label": "autophagosome membrane",
  "gene_name": "Microtubule-associated proteins 1A_1B light chain 3B",
  "gene_symbol": "MAP1LC3B"
}